{
  "gene_name": "Integrin alpha-4",
  "gene": "UniProtKB:P13612",
  "gene_symbol": "ITGA4",
  "term_label": "cell surface",
  "term_id": "GO:0009986"
}